positive regulation of mammary gland involution [GO:1903521] (biological process) Definition: Any process that activates or increases the frequency, rate or extent of mammary gland involution. Also known as: up regulation of mammary gland involution, up-regulation of mammary gland involution, upregulation of mammary gland involution, activation of mammary gland involution References: PMID:23164222 Sources: GOC:TermGenie, GOC:dph, GO_REF:0000058 Relationships: is a type of GO:0034105; is a type of regulation of mammary gland involution [GO:1903519]; positively regulates mammary gland involution [GO:0060056]